positive regulation of hair placode formation [GO:0061169] (biological process) Relationships: is a type of GO:0051094; is a type of regulation of hair follicle placode formation [GO:0061168]; positively regulates hair follicle placode formation [GO:0060789] Sources: GOC:dph Definition: Any process that increases the rate, frequency, or extent of hair follicle placode formation, the developmental process in which a hair placode forms. An hair follicle placode is a thickening of the ectoderm that will give rise to the hair follicle bud.